{
  "term_label": "rDNA heterochromatin",
  "term_id": "GO:0033553",
  "gene": "UniProtKB:Q96EB6",
  "gene_symbol": "SIRT1",
  "gene_name": "NAD-dependent protein deacetylase sirtuin-1"
}